{
  "term_id": "GO:0000086",
  "gene": "UniProtKB:Q8IWQ3",
  "gene_name": "Serine_threonine-protein kinase BRSK2",
  "term_label": "G2/M transition of mitotic cell cycle",
  "gene_symbol": "BRSK2"
}